{
  "gene": "UniProtKB:Q8TAL6",
  "gene_symbol": "FIBIN",
  "term_label": "Unknown cellular component",
  "term_id": "UNKNOWN:0003",
  "gene_name": "Fin bud initiation factor homolog"
}